{
  "term_id": "GO:0007155",
  "gene": "UniProtKB:Q9Y5G7",
  "term_label": "cell adhesion",
  "gene_symbol": "PCDHGA6",
  "gene_name": "Protocadherin gamma-A6"
}